formation of translation initiation ternary complex [GO:0001677] (BP) Definition: Formation of a complex between aminoacylated initiator methionine tRNA, GTP, and initiation factor 2 (either eIF2 in eukaryotes, or IF2 in prokaryotes). In prokaryotes, fMet-tRNA (initiator) is used rather than Met-tRNA (initiator). Sources: GOC:hjd Also known as: translation initiation ternary complex assembly Relationships: is a type of GO:0022618; is part of translational initiation [GO:0006413] Regulation: RO_0002211 by regulation of formation of translation initiation ternary complex [GO:1901190]; negatively regulated by negative regulation of formation of translation initiation ternary complex [GO:1901191]; positively regulated by positive regulation of formation of translation initiation ternary complex [GO:1901192]